{
  "gene": "UniProtKB:O00445",
  "gene_name": "Synaptotagmin-5",
  "gene_symbol": "SYT5",
  "term_label": "vesicle-mediated transport",
  "term_id": "GO:0016192"
}